{
  "gene": "UniProtKB:Q9HDC5",
  "gene_name": "Junctophilin-1",
  "gene_symbol": "JPH1",
  "term_label": "Unknown biological process",
  "term_id": "UNKNOWN:0002"
}